{
  "gene_symbol": "PHF8",
  "gene_name": "Histone lysine demethylase PHF8",
  "term_id": "GO:0006338",
  "term_label": "chromatin remodeling",
  "gene": "UniProtKB:Q9UPP1"
}